{
  "term_id": "GO:0006874",
  "gene": "UniProtKB:Q8IWX8",
  "gene_symbol": "CHERP",
  "term_label": "intracellular calcium ion homeostasis",
  "gene_name": "Calcium homeostasis endoplasmic reticulum protein"
}